regulation of ergot alkaloid biosynthetic process [GO:1900822] (BP) Relationships: is a type of GO:1900376; RO_0002211 ergot alkaloid biosynthetic process [GO:0035837] Definition: Any process that modulates the frequency, rate or extent of ergot alkaloid biosynthetic process. Subtypes: GO:1900646, negative regulation of ergot alkaloid biosynthetic process [GO:1900823], GO:1900824, regulation of fumigaclavine C biosynthetic process [GO:1900837] Sources: GOC:TermGenie, GOC:di Also known as: regulation of ergot alkaloid anabolism, regulation of ergot alkaloid biosynthesis, regulation of ergot alkaloid formation, regulation of ergot alkaloid synthesis